luteolysis [GO:0001554] (BP) Definition: The lysis or structural demise of the corpus luteum. During normal luteolysis, two closely related events occur. First, there is loss of the capacity to synthesize and secrete progesterone (functional luteolysis) followed by loss of the cells that comprise the corpus luteum (structural luteolysis). Preventing luteolysis is crucial to maintain pregnancy. References: PMID:10617764 Relationships: is a type of ovulation cycle process [GO:0022602]; is part of female gonad development [GO:0008585]